{
  "gene": "UniProtKB:Q8NGN0",
  "gene_name": "Olfactory receptor 4D5",
  "term_label": "Unknown biological process",
  "term_id": "UNKNOWN:0002",
  "gene_symbol": "OR4D5"
}